{
  "term_label": "lipid storage",
  "term_id": "GO:0019915",
  "gene_name": "Fat storage-inducing transmembrane protein 1",
  "gene_symbol": "FITM1",
  "gene": "UniProtKB:A5D6W6"
}